L-glutamine:sodium symporter activity [GO:0140902] (molecular function) References: PMID:28416685 Definition: Enables the transfer of a solute or solutes from one side of a membrane to the other according to the reaction: L-glutamine(out) + Na+(out) = L-glutamine(in) + Na+(in). Also known as: glutamine:sodium symporter activity, sodium:L-glutamine symporter activity, sodium:glutamine symporter activity Relationships: is a type of GO:0005295; is a type of GO:0015186; is a type of alanine:sodium symporter activity [GO:0015655]